{
  "gene": "UniProtKB:P06213",
  "gene_name": "Insulin receptor",
  "term_id": "GO:0005886",
  "term_label": "plasma membrane",
  "gene_symbol": "INSR"
}